{
  "term_id": "GO:0042761",
  "term_label": "very long-chain fatty acid biosynthetic process",
  "gene_name": "Trans-2,3-enoyl-CoA reductase-like",
  "gene": "UniProtKB:Q5HYJ1",
  "gene_symbol": "TECRL"
}